allantoin metabolic process [GO:0000255] (biological process) Definition: The chemical reactions and pathways involving allantoin, (2,5-dioxo-4-imidazolidinyl)urea, an intermediate or end product of purine catabolism. Subtypes: allantoin catabolic process [GO:0000256], allantoin biosynthetic process [GO:0019428] Also known as: allantoin metabolism Sources: GOC:mah, ISBN:0198547684 Relationships: is a type of amide metabolic process [GO:0043603]